{
  "term_id": "GO:0000785",
  "gene_symbol": "KDM4B",
  "term_label": "chromatin",
  "gene_name": "Lysine-specific demethylase 4B",
  "gene": "UniProtKB:O94953"
}